{
  "term_label": "cellular response to cytokine stimulus",
  "term_id": "GO:0071345",
  "gene": "UniProtKB:P09913",
  "gene_name": "Interferon-induced protein with tetratricopeptide repeats 2",
  "gene_symbol": "IFIT2"
}